{
  "gene_symbol": "CPEB4",
  "gene_name": "Cytoplasmic polyadenylation element-binding protein 4",
  "term_id": "GO:0043005",
  "gene": "UniProtKB:Q17RY0",
  "term_label": "neuron projection"
}